guanyl nucleotide exchange factor activator activity [GO:0160124] (molecular function) Definition: Binds to and increases the activity of a guanyl nucleotide exchange factor. Relationships: is_a enzyme activator activity [GO:0008047] References: PMID:37463208